lipid oxidation [GO:0034440] (biological process) Relationships: is a type of GO:0030258 Definition: The removal of one or more electrons from a lipid, with or without the concomitant removal of a proton or protons, by reaction with an electron-accepting substance, by addition of oxygen or by removal of hydrogen. Sources: GOC:BHF, GOC:mah Subtypes: fatty acid oxidation [GO:0019395], lipoprotein lipid oxidation [GO:0034439], GO:0080064, GO:0080065